regulation of siRNA-mediated facultative heterochromatin formation [GO:1902802] (biological process) References: PMID:24210919 Sources: GOC:TermGenie, GO_REF:0000058 Relationships: is a type of regulation of regulatory ncRNA-mediated heterochromatin formation [GO:0010964]; regulates siRNA-mediated facultative heterochromatin formation [GO:1902795] Definition: Any process that modulates the frequency, rate or extent of siRNA-dependent facultative heterochromatin formation. Also known as: regulation of HOOD assembly, regulation of HOOD formation, regulation of heterochromatin domain assembly, regulation of heterochromatin domain formation, regulation of siRNA-dependent facultative heterochromatin assembly, regulation of siRNA-dependent facultative heterochromatin formation